gas vesicle shell [GO:0033172] (cellular component) Definition: The proteinaceous structure surrounding a gas vesicle. Sources: GOC:ecd Also known as: gas vesicle wall, gas vesicle membrane Relationships: is a type of cellular anatomical structure [GO:0110165]; is part of GO:0031411